subapical part of cell [GO:0120219] (cellular component) Relationships: is a type of cellular anatomical structure [GO:0110165] Definition: The region of a polarized cell that is just below the apical region. For example, in a polarized epithelial cell, the apical region has an exposed surface and lies opposite to the basal lamina that separates the epithelium from other tissue so the subapical region is further from the exposed surface and closer to the basal lamina. Also known as: subapical region of cell References: PMID:29891944 Sources: GOC:krc